mesonephric connecting tubule development [GO:0061272] (biological process) Also known as: mesonephric collecting tubule development, mesonephric connecting duct development Relationships: is a type of mesonephric nephron tubule development [GO:0061242]; is a type of connecting tubule development [GO:0072027] Definition: The process whose specific outcome is the progression of the mesonephric connecting tubule over time, from its formation to the mature structure. The mesonephric connecting tubule is a tubular segment of the mesonephric nephron; it connects the distal tubule to the collecting duct in the mesonephros. Sources: GOC:mtg_kidney_jan10